{
  "gene_name": "Uncharacterized protein C9orf57",
  "gene_symbol": "C9orf57",
  "term_id": "UNKNOWN:0003",
  "gene": "UniProtKB:Q5W0N0",
  "term_label": "Unknown cellular component"
}